{
  "gene_symbol": "VIM",
  "term_id": "GO:0005882",
  "gene": "UniProtKB:P08670",
  "gene_name": "Vimentin",
  "term_label": "intermediate filament"
}